{
  "term_label": "regulation of transcription by RNA polymerase II",
  "gene_name": "Krueppel-like factor 7",
  "gene_symbol": "KLF7",
  "term_id": "GO:0006357",
  "gene": "UniProtKB:O75840"
}